acyl-lysine deacylase activity [GO:0050477] (molecular function) Definition: Catalysis of the reaction: H2O + N6-acyl-L-lysine = L-lysine + a carboxylate. Sources: EC:3.5.1.17 Also known as: 6-N-acyl-L-lysine amidohydrolase activity, N6-acyl-L-lysine amidohydrolase activity, epsilon-lysine acylase activity Relationships: is a type of GO:0016811